regulation of gamma-delta T cell differentiation [GO:0045586] (biological process) Relationships: is a type of regulation of T cell differentiation [GO:0045580]; is a type of GO:0046643; RO_0002211 gamma-delta T cell differentiation [GO:0042492] Note: Note that immunologists typically use the word 'development' to refer to cells of B or T cell lineages undergoing the process that GO describes as 'cell differentiation'. Sources: GOC:go_curators Subtypes: negative regulation of gamma-delta T cell differentiation [GO:0045587], positive regulation of gamma-delta T cell differentiation [GO:0045588] Also known as: regulation of gamma-delta T lymphocyte differentiation, regulation of gamma-delta T-cell differentiation, regulation of gamma-delta T-lymphocyte differentiation, regulation of gamma-delta T cell development Definition: Any process that modulates the frequency, rate or extent of gamma-delta T cell differentiation.